regulation of glucosinolate biosynthetic process [GO:0010439] (biological process) Relationships: is a type of regulation of sulfur metabolic process [GO:0042762]; is a type of GO:0043255; is a type of GO:0062012; regulates GO:0019761 Definition: Any process that modulates the frequency, rate or extent of the chemical reactions and pathways resulting in the formation of glucosinolates, substituted thioglucosides found in rapeseed products and related cruciferae. References: PMID:17420480